{
  "gene_symbol": "TMEM44",
  "gene_name": "Transmembrane protein 44",
  "gene": "UniProtKB:Q2T9K0",
  "term_id": "UNKNOWN:0002",
  "term_label": "Unknown biological process"
}